{
  "gene_symbol": "ANKLE1",
  "gene_name": "Ankyrin repeat and LEM domain-containing protein 1",
  "gene": "UniProtKB:Q8NAG6",
  "term_label": "double-strand break repair via homologous recombination",
  "term_id": "GO:0000724"
}